{
  "gene": "UniProtKB:Q9Y6F8",
  "term_label": "transcription corepressor activity",
  "gene_symbol": "CDY1B",
  "gene_name": "Testis-specific chromodomain protein Y 1",
  "term_id": "GO:0003714"
}